{
  "gene": "UniProtKB:Q9NYC9",
  "gene_symbol": "DNAH9",
  "gene_name": "Dynein axonemal heavy chain 9",
  "term_label": "minus-end-directed microtubule motor activity",
  "term_id": "GO:0008569"
}